mitotic nuclear division [GO:0140014] (biological process) Sources: ISBN:0198547684 Relationships: is a type of GO:0000280; is a type of mitotic cell cycle process [GO:1903047] Definition: A mitotic cell cycle process comprising the steps by which the nucleus of a eukaryotic cell divides; the process involves condensation of chromosomal DNA into a highly compacted form. Canonically, mitosis produces two daughter nuclei whose chromosome complement is identical to that of the mother cell. Also known as: mitosis Regulation: regulated by GO:0007088; negatively regulated by GO:0045839; positively regulated by positive regulation of mitotic nuclear division [GO:0045840] Subtypes: generative cell mitosis [GO:0055047]